{
  "term_id": "GO:0005730",
  "gene_symbol": "NIP7",
  "gene_name": "60S ribosome subunit biogenesis protein NIP7 homolog",
  "gene": "UniProtKB:Q9Y221",
  "term_label": "nucleolus"
}